{
  "gene_name": "Tumor necrosis factor receptor superfamily member 10C",
  "gene": "UniProtKB:O14798",
  "term_id": "UNKNOWN:0001",
  "term_label": "Unknown molecular function",
  "gene_symbol": "TNFRSF10C"
}